smoothened signaling pathway involved in regulation of cerebellar granule cell precursor cell proliferation [GO:0021938] (biological process) Also known as: hedgehog signaling pathway involved in regulation of granule cell precursor cell proliferation, hh signaling pathway involved in regulation of granule cell precursor cell proliferation, smoothened signalling pathway in regulation of granule cell precursor cell proliferation References: PMID:15157725 Sources: GOC:cls, GOC:dgh, GOC:dph, GOC:jid, GOC:tb Relationships: is a type of GO:0007224 Definition: The series of molecular signals generated as a consequence of activation of the transmembrane protein Smoothened in cerebellar granule cells that contributes to the regulation of proliferation of the cells.